tRNA (uracil(54)-C5)-methyltransferase activity, 5,10-methylenetetrahydrofolate-dependent [GO:0047151] (molecular function) Also known as: methylenetetrahydrofolate-tRNA-(uracil-5-)-methyltransferase (FADH-oxidizing) activity, tRNA (uracil(54)-C(5))-methyltransferase activity, 5,10-methylenetetrahydrofolate-dependent, 5,10-methylenetetrahydrofolate:tRNA (uracil-5-)-methyltransferase activity, 5,10-methylenetetrahydrofolate:tRNA-UPsiC (uracil-5-)-methyl-transferase activity, folate-dependent ribothymidyl synthase activity, methylenetetrahydrofolate-transfer ribonucleate uracil 5-methyltransferase activity Definition: Catalysis of the reaction: 5,10-methylenetetrahydrofolate + tRNA containing uridine at position 54 + FADH + H+ = tetrahydrofolate + tRNA containing ribothymidine at position 54 + FAD+. Relationships: is a type of tRNA (uridine) methyltransferase activity [GO:0016300] Sources: EC:2.1.1.74, MetaCyc:2.1.1.74-RXN